{
  "term_id": "GO:0043495",
  "gene_symbol": "SUN3",
  "gene": "UniProtKB:Q8TAQ9",
  "gene_name": "SUN domain-containing protein 3",
  "term_label": "protein-membrane adaptor activity"
}